{
  "gene": "UniProtKB:P33176",
  "term_id": "GO:0048489",
  "gene_symbol": "KIF5B",
  "term_label": "synaptic vesicle transport",
  "gene_name": "Kinesin-1 heavy chain"
}